{
  "gene_symbol": "EN1",
  "term_label": "neuron differentiation",
  "gene_name": "Homeobox protein engrailed-1",
  "term_id": "GO:0030182",
  "gene": "UniProtKB:Q05925"
}